{
  "gene": "UniProtKB:Q9Y2K9",
  "gene_name": "Syntaxin-binding protein 5-like",
  "gene_symbol": "STXBP5L",
  "term_label": "cytoplasm",
  "term_id": "GO:0005737"
}